mycophenolic acid acyl-glucuronide esterase activity [GO:0102390] (molecular function) Relationships: is a type of carboxylic ester hydrolase activity [GO:0052689] Definition: Catalysis of the reaction: mycophenolic acid O-acyl-glucuronide(1-) + H2O = mycophenolate + H+ + D-glucopyranuronate. Sources: EC:3.1.1.93, GOC:pz